positive regulation of histidine biosynthetic process [GO:0120215] (biological process) Also known as: positive regulation of histidine anabolism, positive regulation of histidine biosynthesis, positive regulation of histidine formation, positive regulation of histidine synthesis, up regulation of histidine anabolism, up regulation of histidine biosynthesis, up regulation of histidine biosynthetic process, up regulation of histidine formation, up regulation of histidine synthesis, up-regulation of histidine anabolism, up-regulation of histidine biosynthesis, up-regulation of histidine biosynthetic process, up-regulation of histidine formation, up-regulation of histidine synthesis, upregulation of histidine anabolism, upregulation of histidine biosynthesis, upregulation of histidine biosynthetic process, upregulation of histidine formation, upregulation of histidine synthesis, activation of histidine anabolism, activation of histidine biosynthesis, activation of histidine biosynthetic process, activation of histidine formation, activation of histidine synthesis Relationships: is_a positive regulation of small molecule metabolic process [GO:0062013]; is a type of regulation of histidine biosynthetic process [GO:0120213]; is a type of positive regulation of amino acid biosynthetic process [GO:2000284]; positively regulates L-histidine biosynthetic process [GO:0000105] Definition: Any process that activates or increases the frequency, rate or extent of histidine biosynthetic process. Sources: GOC:krc